negative regulation by host of viral glycoprotein metabolic process [GO:0044871] (biological process) Relationships: is a type of host-mediated suppression of viral proces [GO:0044793]; is a type of modulation by host of viral glycoprotein metabolic process [GO:0044870]; is a type of negative regulation of viral process [GO:0048525]; is a type of negative regulation of glycoprotein metabolic process [GO:1903019] Sources: GOC:jl Definition: A process in which a host organism stops, prevents or reduces the frequency, rate or extent of viral glycoprotein metabolic process.